L-proline transmembrane transport [GO:1904555] (BP) Definition: The directed movement of L-proline across a membrane. Subtypes: L-proline import across plasma membrane [GO:1904271] Relationships: is_a proline transport [GO:0015824]; is a type of proline transmembrane transport [GO:0035524]; is_a GO:1902475 Sources: GOC:TermGenie, GOC:kmv, GO_REF:0000069